{
  "gene_symbol": "PRDM9",
  "gene": "UniProtKB:Q9NQV7",
  "term_id": "GO:0005634",
  "term_label": "nucleus",
  "gene_name": "Histone-lysine N-methyltransferase PRDM9"
}